{
  "term_id": "UNKNOWN:0001",
  "term_label": "Unknown molecular function",
  "gene_symbol": "KIAA1328",
  "gene": "UniProtKB:Q86T90",
  "gene_name": "Protein hinderin"
}